{
  "gene_name": "Casein kinase II subunit alpha 3",
  "gene": "UniProtKB:Q8NEV1",
  "gene_symbol": "CSNK2A3",
  "term_label": "double-strand break repair",
  "term_id": "GO:0006302"
}